{
  "gene": "UniProtKB:P21127",
  "term_id": "UNKNOWN:0002",
  "gene_name": "Cyclin-dependent kinase 11B",
  "gene_symbol": "CDK11B",
  "term_label": "Unknown biological process"
}